regulation of phospholipid catabolic process [GO:0060696] (biological process) Definition: Any process that modulates the rate, frequency, or extent of phospholipid catabolism, the chemical reactions and pathways resulting in the breakdown of phospholipids, any lipid containing phosphoric acid as a mono- or diester. Sources: GOC:BHF, GOC:dph, GOC:tb Relationships: is a type of regulation of lipid catabolic process [GO:0050994]; is a type of regulation of phospholipid metabolic process [GO:1903725]; regulates phospholipid catabolic process [GO:0009395] Subtypes: regulation of phosphatidylcholine catabolic process [GO:0010899], GO:0060697, GO:1902641, regulation of sphingomyelin catabolic process [GO:2000754]